{
  "term_id": "GO:0015030",
  "gene": "UniProtKB:Q9BUR4",
  "term_label": "Cajal body",
  "gene_name": "Telomerase Cajal body protein 1",
  "gene_symbol": "WRAP53"
}